platelet activating factor receptor binding [GO:0031859] (molecular function) Definition: Binding to a platelet activating factor receptor. Sources: GOC:mah, GOC:nln Also known as: platelet activating factor receptor ligand Relationships: is a type of G protein-coupled receptor binding [GO:0001664]